{
  "term_id": "UNKNOWN:0002",
  "gene": "UniProtKB:Q7Z5L0",
  "gene_name": "Vitelline membrane outer layer protein 1 homolog",
  "gene_symbol": "VMO1",
  "term_label": "Unknown biological process"
}